{
  "gene": "UniProtKB:P30414",
  "term_id": "GO:0006457",
  "gene_name": "NK-tumor recognition protein",
  "term_label": "protein folding",
  "gene_symbol": "NKTR"
}